{
  "gene_name": "Basigin",
  "gene_symbol": "BSG",
  "term_label": "cell-cell adhesion mediator activity",
  "term_id": "GO:0098632",
  "gene": "UniProtKB:P35613"
}